{
  "term_label": "liver development",
  "gene_symbol": "UGT1A1",
  "term_id": "GO:0001889",
  "gene": "UniProtKB:P22309",
  "gene_name": "UDP-glucuronosyltransferase 1A1"
}